{
  "gene_name": "Spindle and kinetochore-associated protein 1",
  "gene": "UniProtKB:Q96BD8",
  "gene_symbol": "SKA1",
  "term_id": "GO:0005876",
  "term_label": "spindle microtubule"
}